hair follicle morphogenesis [GO:0031069] (BP) Definition: The process in which the anatomical structures of the hair follicle are generated and organized. Sources: GOC:ln Relationships: is a type of anatomical structure morphogenesis [GO:0009653]; is a type of hair cycle process [GO:0022405]; is part of GO:0001942; is part of epidermis morphogenesis [GO:0048730]